snRNA 3'-end processing [GO:0034472] (biological process) Also known as: snRNA 3' end processing Relationships: is a type of snRNA processing [GO:0016180]; is_a RNA 3'-end processing [GO:0031123] Definition: Any process involved in forming the mature 3' end of an snRNA molecule. Subtypes: U1 snRNA 3'-end processing [GO:0034473], U2 snRNA 3'-end processing [GO:0034474], U4 snRNA 3'-end processing [GO:0034475], GO:0034476, U6 snRNA 3'-end processing [GO:0034477] Sources: GOC:mah